{
  "term_id": "GO:0045727",
  "gene_symbol": "FXR2",
  "term_label": "positive regulation of translation",
  "gene": "UniProtKB:P51116",
  "gene_name": "RNA-binding protein FXR2"
}